{
  "gene_name": "ADP-ribosylation factor-like protein 13B",
  "term_id": "GO:0031514",
  "gene_symbol": "ARL13B",
  "gene": "UniProtKB:Q3SXY8",
  "term_label": "motile cilium"
}